{
  "gene_name": "Cytoplasmic dynein 2 intermediate chain 2",
  "gene": "UniProtKB:Q96EX3",
  "term_label": "cytoplasmic dynein complex",
  "term_id": "GO:0005868",
  "gene_symbol": "DYNC2I2"
}